{
  "gene_name": "Pancreas transcription factor 1 subunit alpha",
  "term_id": "GO:0032502",
  "term_label": "developmental process",
  "gene": "UniProtKB:Q7RTS3",
  "gene_symbol": "PTF1A"
}